{
  "gene": "UniProtKB:Q15622",
  "term_id": "GO:0007165",
  "gene_symbol": "OR7A5",
  "gene_name": "Olfactory receptor 7A5",
  "term_label": "signal transduction"
}